{
  "gene_name": "Actin-binding protein WASF3",
  "gene_symbol": "WASF3",
  "gene": "UniProtKB:Q9UPY6",
  "term_label": "SCAR complex",
  "term_id": "GO:0031209"
}